{
  "term_label": "Unknown cellular component",
  "gene_symbol": "TMEM273",
  "gene_name": "Transmembrane protein 273",
  "term_id": "UNKNOWN:0003",
  "gene": "UniProtKB:Q5T292"
}